chaeta development [GO:0022416] (biological process) Subtypes: cibarial fish-trap bristle development [GO:0048725] Definition: The process whose specific outcome is the progression of a chaeta over time, from its formation to the mature structure. A chaeta is a sensory multicellular cuticular outgrowth of a specifically differentiated cell. Also known as: bristle development Relationships: is a type of GO:0007423 Sources: FBbt:00005177, GOC:bf, GOC:cjm, GOC:dos, GOC:isa_complete